negative regulation of protein lipidation [GO:1903060] (biological process) Subtypes: GO:0060262, negative regulation of peptidyl-L-cysteine S-palmitoylation [GO:1902663] Relationships: is_a GO:0010558; is a type of negative regulation of protein modification process [GO:0031400]; is a type of negative regulation of lipoprotein metabolic process [GO:0050748]; is a type of regulation of protein lipidation [GO:1903059]; RO_0002212 protein lipidation [GO:0006497] Definition: Any process that stops, prevents or reduces the frequency, rate or extent of protein lipidation. Also known as: down regulation of lipid:protein modification, down regulation of protein amino acid lipidation, down regulation of protein lipidation, down-regulation of lipid:protein modification, down-regulation of protein amino acid lipidation, down-regulation of protein lipidation, downregulation of lipid:protein modification, downregulation of protein amino acid lipidation, downregulation of protein lipidation, negative regulation of lipid:protein modification, negative regulation of protein amino acid lipidation, inhibition of lipid:protein modification, inhibition of protein amino acid lipidation, inhibition of protein lipidation References: PMID:21909394 Sources: GOC:TermGenie, GOC:rph, GO_REF:0000058